{
  "gene_name": "Probable G-protein coupled receptor 85",
  "term_label": "Unknown biological process",
  "gene": "UniProtKB:P60893",
  "gene_symbol": "GPR85",
  "term_id": "UNKNOWN:0002"
}